{
  "term_label": "vesicle-mediated transport",
  "gene": "UniProtKB:P61966",
  "gene_name": "AP-1 complex subunit sigma-1A",
  "gene_symbol": "AP1S1",
  "term_id": "GO:0016192"
}